{
  "term_id": "UNKNOWN:0002",
  "term_label": "Unknown biological process",
  "gene_name": "Putative uncharacterized protein FLJ37218",
  "gene": "UniProtKB:Q8N1Y9",
  "gene_symbol": "Q8N1Y9"
}